positive regulation of cardiac chamber morphogenesis [GO:1901221] (biological process) Sources: GOC:BHF, GOC:TermGenie Relationships: is a type of positive regulation of developmental process [GO:0051094]; is a type of regulation of cardiac chamber morphogenesis [GO:1901219]; positively regulates cardiac chamber morphogenesis [GO:0003206] Also known as: positive regulation of heart chamber morphogenesis, up regulation of cardiac chamber morphogenesis, up regulation of heart chamber morphogenesis, up-regulation of cardiac chamber morphogenesis, up-regulation of heart chamber morphogenesis, upregulation of cardiac chamber morphogenesis, upregulation of heart chamber morphogenesis, activation of cardiac chamber morphogenesis, activation of heart chamber morphogenesis Definition: Any process that activates or increases the frequency, rate or extent of cardiac chamber morphogenesis. Subtypes: positive regulation of cardiac chamber formation [GO:1901212]